anterior neuropore closure [GO:0021506] (biological process) Definition: The joining together of the neural folds of the rostral opening of the neural tube. The anterior neuropore appears before the process of neural tube closure is complete. Sources: GOC:cls, GOC:dgh, GOC:dph, GOC:jid, GO_REF:0000021 Relationships: is a type of morphogenesis of embryonic epithelium [GO:0016331]; is part of neuropore closure [GO:0021995]